{
  "gene_name": "Forkhead box protein E3",
  "term_id": "GO:0030154",
  "gene": "UniProtKB:Q13461",
  "term_label": "cell differentiation",
  "gene_symbol": "FOXE3"
}